{
  "gene_symbol": "KIF2A",
  "gene": "UniProtKB:O00139",
  "term_label": "ATP hydrolysis activity",
  "term_id": "GO:0016887",
  "gene_name": "Kinesin-like protein KIF2A"
}